regulation of sulfate assimilation [GO:1900058] (biological process) Definition: Any process that modulates the frequency, rate or extent of sulfate assimilation. Relationships: is a type of regulation of sulfur metabolic process [GO:0042762]; regulates GO:0000103 Subtypes: positive regulation of sulfate assimilation [GO:1900059] Also known as: regulation of sulphate assimilation, regulation of sulfate assimilation, phosphoadenylyl sulfate reduction by an oxidoreductase, acting on sulfur group of donors, NAD or NADP as acceptor, regulation of sulphate assimilation, phosphoadenylyl sulphate reduction by an oxidoreductase, acting on sulphur group of donors, NAD or NADP as acceptor References: PMID:7601277, PMID:7891681 Sources: GOC:TermGenie